{
  "term_label": "mitotic cytokinesis",
  "gene": "UniProtKB:P23528",
  "gene_name": "Cofilin-1",
  "term_id": "GO:0000281",
  "gene_symbol": "CFL1"
}